pyramidal neuron migration to cerebral cortex [GO:0021852] (biological process) Definition: The migration of a pyramidal neuron precursor from the ventricular zone to the correct layer of the cerebral cortex. References: PMID:12626695, PMID:22192824 Sources: GOC:cls, GOC:dgh, GOC:dph, GOC:jid, GO_REF:0000021 Also known as: pyramidal neuron migration, projection neuron migration Relationships: is a type of cerebral cortex radial glia-guided migration [GO:0021801]; is a type of radial glia-guided pyramidal neuron migration [GO:0140650]; is part of GO:0021860